{
  "gene": "UniProtKB:Q8NAM6",
  "gene_symbol": "ZSCAN4",
  "gene_name": "Zinc finger and SCAN domain-containing protein 4",
  "term_id": "GO:0006357",
  "term_label": "regulation of transcription by RNA polymerase II"
}